homophilic cell-cell adhesion [GO:0007156] (biological process) Regulation: regulated by regulation of homophilic cell adhesion [GO:1903385]; negatively regulated by negative regulation of homophilic cell adhesion [GO:1903386]; positively regulated by positive regulation of homophilic cell adhesion [GO:1903387] Definition: The attachment of an adhesion molecule in one cell to an identical molecule in an adjacent cell. Relationships: is a type of cell-cell adhesion [GO:0098609] Sources: ISBN:0198506732